{
  "term_label": "ubiquitin protein ligase activity",
  "gene": "UniProtKB:Q99728",
  "gene_name": "BRCA1-associated RING domain protein 1",
  "term_id": "GO:0061630",
  "gene_symbol": "BARD1"
}